{
  "term_id": "GO:0005769",
  "gene": "UniProtKB:P51148",
  "gene_symbol": "RAB5C",
  "gene_name": "Ras-related protein Rab-5C",
  "term_label": "early endosome"
}